{
  "gene_symbol": "TMEM150A",
  "term_id": "GO:0005886",
  "gene": "UniProtKB:Q86TG1",
  "gene_name": "Transmembrane protein 150A",
  "term_label": "plasma membrane"
}